{
  "gene_name": "Syndetin",
  "term_label": "endocytic recycling",
  "term_id": "GO:0032456",
  "gene": "UniProtKB:Q96JG6",
  "gene_symbol": "VPS50"
}